protein serine/threonine kinase inhibitor activity [GO:0030291] (molecular function) Relationships: is a type of GO:0004860; negatively regulates protein serine/threonine kinase activity [GO:0004674] Definition: Binds to and stops, prevents or reduces the activity of a protein serine/threonine kinase. Sources: GOC:mah Subtypes: cyclin-dependent protein serine/threonine kinase inhibitor activity [GO:0004861], cAMP-dependent protein kinase inhibitor activity [GO:0004862], GO:0008426, calcium-dependent protein kinase inhibitor activity [GO:0008427]